{
  "term_label": "lysosome",
  "term_id": "GO:0005764",
  "gene_symbol": "LAMTOR5",
  "gene": "UniProtKB:O43504",
  "gene_name": "Ragulator complex protein LAMTOR5"
}